peptide N-succinyltransferase activity [GO:0106075] (molecular function) Definition: Catalysis of the acetylation of an amino acid residue of a peptide or protein, according to the reaction: succinyl-CoA + peptide = CoA + N-succinylpeptide. Relationships: is a type of GO:0016410 Subtypes: peptide-lysine-N-succinyltransferase activity [GO:0106076], histone succinyltransferase activity [GO:0106078] References: PMID:29211711